{
  "gene_name": "P2Y purinoceptor 8",
  "term_id": "GO:0004930",
  "gene_symbol": "P2RY8",
  "gene": "UniProtKB:Q86VZ1",
  "term_label": "G protein-coupled receptor activity"
}